{
  "gene_name": "Endothelial cell-selective adhesion molecule",
  "gene_symbol": "ESAM",
  "term_label": "plasma membrane",
  "gene": "UniProtKB:Q96AP7",
  "term_id": "GO:0005886"
}